{
  "gene_symbol": "DPY19L3",
  "gene_name": "Probable C-mannosyltransferase DPY19L3",
  "term_label": "Unknown biological process",
  "term_id": "UNKNOWN:0002",
  "gene": "UniProtKB:Q6ZPD9"
}